{
  "term_label": "Unknown molecular function",
  "term_id": "UNKNOWN:0001",
  "gene": "UniProtKB:A0A1B0GW54",
  "gene_symbol": "SMIM39",
  "gene_name": "Small integral membrane protein 39"
}